{
  "term_label": "spindle",
  "term_id": "GO:0005819",
  "gene_name": "Katanin p60 ATPase-containing subunit A-like 2",
  "gene_symbol": "KATNAL2",
  "gene": "UniProtKB:Q8IYT4"
}